{
  "gene_symbol": "NANOS3",
  "term_label": "mRNA binding",
  "gene_name": "Nanos homolog 3",
  "gene": "UniProtKB:P60323",
  "term_id": "GO:0003729"
}